{
  "gene_symbol": "PARD3",
  "term_label": "apical junction complex",
  "gene_name": "Partitioning defective 3 homolog",
  "gene": "UniProtKB:Q8TEW0",
  "term_id": "GO:0043296"
}